{
  "term_label": "Unknown cellular component",
  "gene_symbol": "CDON",
  "term_id": "UNKNOWN:0003",
  "gene_name": "Cell adhesion molecule-related_down-regulated by oncogenes",
  "gene": "UniProtKB:Q4KMG0"
}